establishment of protein localization to euchromatin [GO:1905633] (biological process) Also known as: establishment of protein localisation in euchromatin, establishment of protein localisation to euchromatin, establishment of protein localization in euchromatin Relationships: is a type of establishment of protein localization to chromatin [GO:0071169] References: PMID:20889714 Sources: GOC:TermGenie, GO_REF:0000087 Definition: The directed movement of a protein to a specific location in an euchromatin.